{
  "term_id": "GO:0140374",
  "term_label": "antiviral innate immune response",
  "gene_name": "Palmitoyltransferase ZDHHC1",
  "gene": "UniProtKB:Q8WTX9",
  "gene_symbol": "ZDHHC1"
}